{
  "gene_name": "Sodium_potassium-transporting ATPase subunit alpha-4",
  "term_id": "GO:0005886",
  "term_label": "plasma membrane",
  "gene_symbol": "ATP1A4",
  "gene": "UniProtKB:Q13733"
}